{
  "gene_symbol": "ZNF518B",
  "term_id": "GO:0005634",
  "gene_name": "Zinc finger protein 518B",
  "gene": "UniProtKB:Q9C0D4",
  "term_label": "nucleus"
}